outer ear unfolding [GO:0060185] (BP) Sources: GOC:dph Definition: The opening and spreading out of the outer ear. Relationships: is a type of anatomical structure arrangement [GO:0048532]; is part of outer ear morphogenesis [GO:0042473]